{
  "gene_symbol": "SIGLEC15",
  "term_id": "UNKNOWN:0001",
  "term_label": "Unknown molecular function",
  "gene_name": "Sialic acid-binding Ig-like lectin 15",
  "gene": "UniProtKB:Q6ZMC9"
}